site-specific DNA-methyltransferase (adenine-specific) activity [GO:0009007] (molecular function) Sources: EC:2.1.1.72 Relationships: is_a GO:0008757; is a type of DNA-methyltransferase activity [GO:0009008] Definition: Catalysis of the reaction: S-adenosyl-L-methionine + DNA adenine = S-adenosyl-L-homocysteine + DNA 6-methylaminopurine. Also known as: DNA adenine methylase, EcoRI methylase, N-6 adenine-specific DNA methylase activity, modification methylase activity, restriction-modification system activity